regulation of septation initiation signaling [GO:0031029] (biological process) Definition: Any process that modulates the frequency, rate or extent of septation initiation signaling. Sources: GOC:mah Also known as: regulation of septation initiation network, regulation of septation initiation signalling, regulation of septation initiation signaling cascade Relationships: is_a regulation of small GTPase mediated signal transduction [GO:0051056]; regulates GO:0031028 Subtypes: negative regulation of septation initiation signaling [GO:0031030], positive regulation of septation initiation signaling [GO:0031031]